{
  "gene_name": "Inverted formin-2",
  "gene_symbol": "INF2",
  "term_id": "UNKNOWN:0001",
  "term_label": "Unknown molecular function",
  "gene": "UniProtKB:Q27J81"
}